{
  "term_label": "synaptic vesicle",
  "gene_symbol": "NGF",
  "term_id": "GO:0008021",
  "gene": "UniProtKB:P01138",
  "gene_name": "Beta-nerve growth factor"
}